interleukin-20 receptor activity [GO:0042016] (molecular function) Also known as: IL-20 receptor activity, IL-20R Definition: Combining with interleukin-20 and transmitting the signal from one side of the membrane to the other to initiate a change in cell activity. Relationships: is_a cytokine receptor activity [GO:0004896]; is part of GO:0140866; has part interleukin-20 binding [GO:0042015] Sources: GOC:jl, GOC:signaling